mitotic nuclear membrane organization [GO:0101024] (biological process) Definition: A mitotic cell cycle process which results in the assembly, arrangement, or disassembly of the nuclear inner or outer membrane during mitosis. Subtypes: mitotic nuclear membrane reassembly [GO:0007084], vesicle fusion with nuclear membrane involved in mitotic nuclear envelope reassembly [GO:0007086], mitotic nuclear bridge organization [GO:0140515] References: PMID:15147872 Sources: GOC:vw Relationships: is a type of nuclear membrane organization [GO:0071763]; is a type of mitotic cell cycle process [GO:1903047]; BFO_0000050 mitotic nuclear division [GO:0140014] Note: This process only occurs in organisms which undergo 'closed mitosis' without nuclear breakdown. Also known as: nuclear membrane organization involved in mitotic nuclear division